{
  "term_label": "Unknown molecular function",
  "gene_symbol": "CYP4F12",
  "gene_name": "Cytochrome P450 4F12",
  "term_id": "UNKNOWN:0001",
  "gene": "UniProtKB:Q9HCS2"
}